{
  "term_id": "GO:0008331",
  "gene": "UniProtKB:Q13698",
  "gene_symbol": "CACNA1S",
  "term_label": "high voltage-gated calcium channel activity",
  "gene_name": "Voltage-dependent L-type calcium channel subunit alpha-1S"
}